lumenal side of endoplasmic reticulum membrane [GO:0098553] (cellular component) Definition: The side (leaflet) of the plasma membrane that faces the lumen. Subtypes: lumenal side of rough endoplasmic reticulum membrane [GO:0098555], GO:0098558 Relationships: is a type of lumenal side of membrane [GO:0098576]; is part of GO:0005789 Sources: GOC:ab, GOC:dos